cellular bud neck septin ring [GO:0000144] (cellular component) References: PMID:16009555 Sources: GOC:krc Relationships: is a type of cellular bud neck septin structure [GO:0000399]; is a type of septin ring [GO:0005940]; is_a cleavage apparatus septin structure [GO:0032161] Definition: A ring-shaped structure that forms at the site of cytokinesis in the bud neck of a budding cell; composed of members of the conserved family of filament forming proteins called septins as well as septin-associated proteins. In S. cerevisiae, this structure forms at the time of bud emergence and the septins show a high rate of exchange.